{
  "term_id": "GO:0005886",
  "gene_symbol": "PCDHA1",
  "gene_name": "Protocadherin alpha-1",
  "gene": "UniProtKB:Q9Y5I3",
  "term_label": "plasma membrane"
}